(22S)-22-hydroxy-campesterol C-23 hydroxylase activity [GO:0102134] (molecular function) Sources: GOC:pz Relationships: is a type of oxidoreductase activity, acting on paired donors, with incorporation or reduction of molecular oxygen, NAD(P)H as one donor, and incorporation of one atom of oxygen [GO:0016709] Definition: Catalysis of the reaction: H+ + (22S)-22-hydroxycampesterol + NADPH + O2 = (22R,23R)-22,23-dihydroxycampesterol + NADP + H2O.